{
  "gene": "UniProtKB:Q16690",
  "gene_symbol": "DUSP5",
  "term_id": "GO:0004721",
  "term_label": "phosphoprotein phosphatase activity",
  "gene_name": "Dual specificity protein phosphatase 5"
}